positive regulation of hormone biosynthetic process [GO:0046886] (biological process) Also known as: positive regulation of hormone anabolism, positive regulation of hormone biosynthesis, positive regulation of hormone formation, positive regulation of hormone synthesis, up regulation of hormone biosynthetic process, up-regulation of hormone biosynthetic process, upregulation of hormone biosynthetic process, activation of hormone biosynthetic process, stimulation of hormone biosynthetic process Sources: GOC:ai Subtypes: GO:0010601, positive regulation of juvenile hormone biosynthetic process [GO:0045969], positive regulation of steroid hormone biosynthetic process [GO:0090031], positive regulation of estrogen biosynthetic process [GO:1904078], GO:2000184 Relationships: is a type of positive regulation of biosynthetic process [GO:0009891]; is a type of positive regulation of hormone metabolic process [GO:0032352]; is a type of GO:0046885; positively regulates hormone biosynthetic process [GO:0042446] Definition: Any process that activates or increases the frequency, rate or extent of the chemical reactions and pathways resulting in the formation of hormones.